{
  "gene_symbol": "CD59",
  "term_label": "negative regulation of activation of membrane attack complex",
  "gene_name": "CD59 glycoprotein",
  "gene": "UniProtKB:P13987",
  "term_id": "GO:0001971"
}